inflammatory response [GO:0006954] (biological process) Subtypes: GO:0002437, acute inflammatory response [GO:0002526], chronic inflammatory response [GO:0002544], pyroptotic inflammatory response [GO:0070269], GO:0090594, neuroinflammatory response [GO:0150076] Sources: GO_REF:0000022, ISBN:0198506732 Definition: The immediate defensive reaction (by vertebrate tissue) to infection or injury caused by chemical or physical agents. The process is characterized by local vasodilation, extravasation of plasma into intercellular spaces and accumulation of white blood cells and macrophages. Relationships: is a type of GO:0006952 Also known as: inflammation Regulation: regulated by regulation of inflammatory response [GO:0050727]; negatively regulated by negative regulation of inflammatory response [GO:0050728]; positively regulated by positive regulation of inflammatory response [GO:0050729]